{
  "term_id": "GO:0031090",
  "gene_symbol": "WLS",
  "gene": "UniProtKB:Q5T9L3",
  "term_label": "organelle membrane",
  "gene_name": "Protein wntless homolog"
}